{
  "gene_symbol": "A0A8V8TLY5",
  "term_id": "UNKNOWN:0001",
  "gene": "UniProtKB:A0A8V8TLY5",
  "gene_name": "Ig-like domain-containing protein (Fragment)",
  "term_label": "Unknown molecular function"
}